{
  "gene_symbol": "OR5K4",
  "gene_name": "Olfactory receptor 5K4",
  "term_label": "Unknown biological process",
  "term_id": "UNKNOWN:0002",
  "gene": "UniProtKB:A6NMS3"
}